{
  "term_id": "UNKNOWN:0003",
  "term_label": "Unknown cellular component",
  "gene_symbol": "PCNT",
  "gene": "UniProtKB:O95613",
  "gene_name": "Pericentrin"
}